{
  "gene": "UniProtKB:Q9H4K1",
  "term_label": "Unknown biological process",
  "term_id": "UNKNOWN:0002",
  "gene_symbol": "RIBC2",
  "gene_name": "RIB43A-like with coiled-coils protein 2"
}